negative regulation of muscle tissue development [GO:1901862] (biological process) Subtypes: negative regulation of striated muscle tissue development [GO:0045843], negative regulation of smooth muscle tissue development [GO:1905900] Also known as: down regulation of muscle tissue development, down-regulation of muscle tissue development, downregulation of muscle tissue development, inhibition of muscle tissue development References: PMID:23150719 Sources: GOC:TermGenie, GOC:yaf Definition: Any process that stops, prevents or reduces the frequency, rate or extent of muscle tissue development. Relationships: is a type of negative regulation of developmental process [GO:0051093]; is_a regulation of muscle tissue development [GO:1901861]; negatively regulates muscle tissue development [GO:0060537]